{
  "term_id": "GO:0043161",
  "gene_symbol": "PRAMEF25",
  "term_label": "proteasome-mediated ubiquitin-dependent protein catabolic process",
  "gene_name": "PRAME family member 25",
  "gene": "UniProtKB:A6NGN4"
}